{
  "gene": "UniProtKB:P55851",
  "term_label": "mitochondrial transmembrane transport",
  "term_id": "GO:1990542",
  "gene_name": "Dicarboxylate carrier SLC25A8",
  "gene_symbol": "UCP2"
}